{
  "term_id": "GO:0005634",
  "gene_symbol": "NOL9",
  "gene_name": "Polynucleotide 5'-hydroxyl-kinase NOL9",
  "gene": "UniProtKB:Q5SY16",
  "term_label": "nucleus"
}